inhibitory neuromuscular junction of somatic myotube [GO:0098526] (cellular component) Relationships: is a type of inhibitory neuromuscular junction [GO:0098521]; is a type of GO:0098524 Sources: GOC:dos Definition: A neuromuscular junction that functions in the inhibition of somatic muscle myotube contraction. Examples of somatic muscle myotubes include the somatic muscle cells of arthropods.